{
  "gene_name": "Leucine-rich repeat-containing protein 14",
  "gene_symbol": "LRRC14",
  "term_label": "cytoplasm",
  "term_id": "GO:0005737",
  "gene": "UniProtKB:Q15048"
}